{
  "term_label": "Golgi apparatus",
  "gene_symbol": "CHPT1",
  "term_id": "GO:0005794",
  "gene": "UniProtKB:Q8WUD6",
  "gene_name": "Cholinephosphotransferase 1"
}